symbiont-mediated suppression of host mRNA processing [GO:0039524] (BP) References: PMID:16571812 Sources: GOC:bf, GOC:sp, VZ:903 Also known as: negative regulation of host mRNA processing, inhibition of host mRNA processing, inhibition by virus of host mRNA processing, inhibition of host pre-mRNA processing by virus, suppression by virus of host mRNA processing Relationships: is a type of symbiont-mediated perturbation of host gene expression [GO:0039656] Definition: A process in which a symbiont inhibits or disrupts mRNA processing in its host. mRNA processing is the conversion of a primary mRNA transcript into one or more mature mRNA(s) prior to translation into polypeptide. The host is defined as the larger of the organisms involved in a symbiotic interaction. Subtypes: symbiont-mediated suppression of host mRNA splicing [GO:0046780]